{
  "term_id": "GO:0099078",
  "gene_symbol": "BORCS5",
  "gene_name": "BLOC-1-related complex subunit 5",
  "gene": "UniProtKB:Q969J3",
  "term_label": "BORC complex"
}